aryl-alcohol dehydrogenase (NAD+) activity [GO:0018456] (molecular function) Relationships: is a type of alcohol dehydrogenase (NAD+) activity [GO:0004022] Also known as: benzyl alcohol dehydrogenase activity, p-hydroxybenzyl alcohol dehydrogenase activity, aryl-alcohol:NAD+ oxidoreductase activity Definition: Catalysis of the reaction: an aromatic alcohol + NAD+ = an aromatic aldehyde + NADH + H+. Sources: EC:1.1.1.90